{
  "term_id": "GO:0032436",
  "gene": "UniProtKB:Q92519",
  "term_label": "positive regulation of proteasomal ubiquitin-dependent protein catabolic process",
  "gene_name": "Tribbles homolog 2",
  "gene_symbol": "TRIB2"
}